{
  "term_id": "UNKNOWN:0003",
  "gene_name": "Solute carrier family 22 member 15",
  "gene_symbol": "SLC22A15",
  "term_label": "Unknown cellular component",
  "gene": "UniProtKB:Q8IZD6"
}